{
  "gene": "UniProtKB:A0A0B4J262",
  "term_label": "adaptive immune response",
  "gene_name": "T cell receptor alpha variable 8-6",
  "gene_symbol": "TRAV8-6",
  "term_id": "GO:0002250"
}